sequestering of BMP from receptor via BMP binding [GO:0038098] (biological process) Relationships: is a type of negative regulation of BMP signaling pathway [GO:0030514]; is a type of GO:0035581 Definition: Binding to a bone morphogenetic protein (BMP) in the extracellular region, and inhibiting BMP signaling by preventing BMP from binding to its cell surface receptor. Also known as: extracellular sequestering of BMP, extracellular sequestering of bone morphogenetic protein References: PMID:19855014 Sources: GOC:bf, GOC:signaling